aflatoxin B synthase activity [GO:0140399] (molecular function) Relationships: is a type of oxidoreductase activity, acting on paired donors, with incorporation or reduction of molecular oxygen, reduced flavin or flavoprotein as one donor, and incorporation of one atom of oxygen [GO:0016712]; is part of aflatoxin biosynthetic process [GO:0045122] Sources: EC:1.14.14.117 Definition: Catalyzes the reaction: 8-O-methylsterigmatocystin + 2 [reduced NADPH--hemoprotein reductase] + 2 O2 = aflatoxin B + 2 [oxidized NADPH--hemoprotein reductase] + H2O + methanol + CO2. Produces both aflatoxin B(1) and aflatoxin B(2).